direct ossification [GO:0036072] (biological process) Relationships: is a type of ossification [GO:0001503] Definition: The formation of bone or of a bony substance, or the conversion of fibrous tissue or of cartilage into bone or a bony substance, that does not require the replacement of preexisting tissues. Sources: GO_REF:0000034 Subtypes: GO:0001957, GO:0036074